{
  "term_label": "Unknown molecular function",
  "gene": "UniProtKB:Q9BY27",
  "gene_symbol": "DGCR6L",
  "term_id": "UNKNOWN:0001",
  "gene_name": "Protein DGCR6L"
}